shikimate metabolic process [GO:0019632] (biological process) Definition: The chemical reactions and pathways involving shikimate, (3R,4S,5R)--3,4,5-trihydroxycyclohex-1-ene-1-carboxylate, the anion of shikimic acid. It is an important intermediate in the biosynthesis of aromatic amino acids. Also known as: shikimate metabolism Subtypes: shikimate catabolic process [GO:0019633] Relationships: is a type of GO:0032787 Sources: GOC:sm, ISBN:0198547684